{
  "gene_symbol": "CHRNA4",
  "term_id": "GO:0022848",
  "gene": "UniProtKB:P43681",
  "gene_name": "Neuronal acetylcholine receptor subunit alpha-4",
  "term_label": "acetylcholine-gated monoatomic cation-selective channel activity"
}